{
  "gene_symbol": "IDE",
  "gene": "UniProtKB:P14735",
  "term_id": "GO:0042447",
  "gene_name": "Insulin-degrading enzyme",
  "term_label": "hormone catabolic process"
}